{
  "term_id": "GO:0009986",
  "gene": "UniProtKB:Q9H4D0",
  "gene_name": "Calsyntenin-2",
  "gene_symbol": "CLSTN2",
  "term_label": "cell surface"
}